regulation of ovulation [GO:0060278] (biological process) Relationships: is a type of regulation of multicellular organismal process [GO:0051239]; is a type of regulation of reproductive process [GO:2000241]; regulates ovulation [GO:0030728] Definition: Any process that modulates the frequency, rate or extent of ovulation, the release of a mature ovum/oocyte from an ovary. Sources: GOC:dph, GOC:kmv, GOC:tb Subtypes: positive regulation of ovulation [GO:0060279], negative regulation of ovulation [GO:0060280]